{
  "gene_name": "Uncharacterized protein C3orf36",
  "gene": "UniProtKB:Q3SXR2",
  "term_id": "UNKNOWN:0003",
  "gene_symbol": "C3orf36",
  "term_label": "Unknown cellular component"
}